{
  "term_id": "GO:0048172",
  "term_label": "regulation of short-term neuronal synaptic plasticity",
  "gene": "UniProtKB:Q6ZSJ9",
  "gene_name": "Protein shisa-6",
  "gene_symbol": "SHISA6"
}